{
  "term_label": "cytokine-mediated signaling pathway",
  "term_id": "GO:0019221",
  "gene_symbol": "JAK3",
  "gene_name": "Tyrosine-protein kinase JAK3",
  "gene": "UniProtKB:P52333"
}